{
  "gene_name": "C-C motif chemokine 4-like",
  "gene": "UniProtKB:Q8NHW4",
  "term_label": "antimicrobial humoral immune response mediated by antimicrobial peptide",
  "term_id": "GO:0061844",
  "gene_symbol": "CCL4L1"
}